{
  "term_id": "GO:0050728",
  "gene_symbol": "AOAH",
  "term_label": "negative regulation of inflammatory response",
  "gene_name": "Acyloxyacyl hydrolase",
  "gene": "UniProtKB:P28039"
}